{
  "gene_symbol": "APOBEC3D",
  "term_label": "negative regulation of single stranded viral RNA replication via double stranded DNA intermediate",
  "term_id": "GO:0045869",
  "gene": "UniProtKB:Q96AK3",
  "gene_name": "DNA dC-dU-editing enzyme APOBEC-3D"
}